{
  "term_label": "L-proline transmembrane transporter activity",
  "term_id": "GO:0015193",
  "gene_name": "Proton-coupled amino acid transporter 3",
  "gene": "UniProtKB:Q495N2",
  "gene_symbol": "SLC36A3"
}